neuropilin signaling pathway [GO:0038189] (biological process) Subtypes: GO:0038190 Definition: The series of molecular signals initiated by an extracellular ligand binding to a neuropilin protein on the surface of a target cell, and ending with the regulation of a downstream cellular process, e.g. transcription. Also known as: Npn signaling References: PMID:12852851 Sources: GOC:BHF Relationships: is a type of GO:0007166